{
  "term_label": "protein folding",
  "gene_symbol": "PPIAL4D",
  "gene": "UniProtKB:F5H284",
  "gene_name": "Peptidyl-prolyl cis-trans isomerase A-like 4D",
  "term_id": "GO:0006457"
}